superinfection exclusion [GO:0098669] (biological process) References: PMID:11985726, PMID:23692331, PMID:24089557, PMID:8012757 Sources: VZ:3971 Relationships: is a type of viral process [GO:0016032] Definition: The process by which a preexisting viral infection prevents a secondary infection with the same or a closely related virus. Typically some aspect of viral entry is inhibited, but post entry mechanisms have also been documented.